{
  "gene_name": "Tubulin gamma-2 chain",
  "gene_symbol": "TUBG2",
  "term_id": "GO:0005634",
  "gene": "UniProtKB:Q9NRH3",
  "term_label": "nucleus"
}